D-glucuronate biosynthetic process [GO:0042841] (biological process) Definition: The chemical reactions and pathways resulting in the formation of D-glucuronate, the D-enantiomer of glucuronate. Relationships: is_a glucuronate biosynthetic process [GO:0046399] Sources: GOC:jl, GOC:jsg, GOC:mah Also known as: D-glucuronate anabolism, D-glucuronate biosynthesis, D-glucuronate formation, D-glucuronate synthesis